{
  "gene_name": "Peroxisome proliferator-activated receptor alpha",
  "gene": "UniProtKB:Q07869",
  "term_id": "GO:0090575",
  "gene_symbol": "PPARA",
  "term_label": "RNA polymerase II transcription regulator complex"
}